{
  "term_id": "GO:0022008",
  "gene_symbol": "FGF5",
  "gene_name": "Fibroblast growth factor 5",
  "gene": "UniProtKB:P12034",
  "term_label": "neurogenesis"
}